{
  "gene": "UniProtKB:P50993",
  "term_label": "sodium ion export across plasma membrane",
  "term_id": "GO:0036376",
  "gene_symbol": "ATP1A2",
  "gene_name": "Sodium_potassium-transporting ATPase subunit alpha-2"
}